{
  "term_id": "GO:0042391",
  "gene_symbol": "KCNH8",
  "gene_name": "Potassium voltage-gated channel subfamily H member 8",
  "gene": "UniProtKB:Q96L42",
  "term_label": "regulation of membrane potential"
}